{
  "term_id": "GO:0005737",
  "term_label": "cytoplasm",
  "gene_symbol": "DUSP21",
  "gene_name": "Dual specificity protein phosphatase 21",
  "gene": "UniProtKB:Q9H596"
}